purine nucleosidase activity [GO:0008477] (molecular function) Also known as: nucleosidase activity, nucleoside hydrolase activity, purine nucleosidase reaction, inosine-adenosine-guanosine preferring nucleoside hydrolase activity, nucleosidase g activity, IAG-NH activity, IAG-nucleoside hydrolase activity, N-D-ribosylpurine ribohydrolase activity, N-ribosyl purine ribohydrolase activity, purine beta-ribosidase activity, purine nucleoside hydrolase activity, purine ribonucleosidase activity, purine-nucleoside ribohydrolase activity, purine-specific nucleoside N-ribohydrolase activity, ribonucleoside hydrolase activity Sources: EC:3.2.2.1 Relationships: is a type of GO:0016799 Definition: Catalysis of the reaction: a N-D-ribosylpurine + H2O = a purine + D-ribose. Subtypes: methylthioadenosine nucleosidase activity [GO:0008930], GO:0047622, inosine nucleosidase activity [GO:0047724], xanthosine nucleotidase activity [GO:0072585], queuosine nucleosidase activity [GO:0106432]